{
  "term_label": "DNA-templated DNA replication",
  "term_id": "GO:0006261",
  "gene": "UniProtKB:Q9NRG0",
  "gene_symbol": "CHRAC1",
  "gene_name": "Chromatin accessibility complex protein 1"
}